FMN catabolic process [GO:0032363] (biological process) Definition: The chemical reactions and pathways resulting in the breakdown of FMN, riboflavin 5'-(dihydrogen phosphate), a coenzyme for a number of oxidative enzymes including NADH dehydrogenase. Sources: GOC:mah Relationships: is a type of ribonucleoside monophosphate catabolic process [GO:0009158]; is a type of ribonucleotide catabolic process [GO:0009261]; is a type of flavin-containing compound catabolic process [GO:0042728]; is a type of FMN metabolic process [GO:0046444]